{
  "term_id": "GO:0005634",
  "term_label": "nucleus",
  "gene_symbol": "S100A5",
  "gene_name": "Protein S100-A5",
  "gene": "UniProtKB:P33763"
}